receptor signaling protein tyrosine kinase inhibitor activity [GO:0030294] (molecular function) Also known as: receptor signalling protein tyrosine kinase inhibitor activity Definition: Stops, prevents or reduces the activity of a receptor signaling protein tyrosine kinase. Sources: GOC:mah Relationships: is a type of protein tyrosine kinase inhibitor activity [GO:0030292]